{
  "gene_symbol": "FATE1",
  "term_id": "GO:0005741",
  "term_label": "mitochondrial outer membrane",
  "gene": "UniProtKB:Q969F0",
  "gene_name": "Fetal and adult testis-expressed transcript protein"
}